{
  "gene": "UniProtKB:P19544",
  "gene_name": "Wilms tumor protein",
  "term_label": "nucleus",
  "gene_symbol": "WT1",
  "term_id": "GO:0005634"
}